anthocyanin 5-O-glucoside-4'''-O-malonyltransferase activity [GO:0102801] (molecular function) Sources: GOC:pz, RHEA:35515 Definition: Catalysis of the reaction: 4'''-demalonylsalvianin + malonyl-CoA = salvianin + coenzyme A. Relationships: is a type of acyltransferase activity, transferring groups other than amino-acyl groups [GO:0016747]